{
  "term_label": "RNA polymerase II cis-regulatory region sequence-specific DNA binding",
  "gene_name": "Zinc finger protein 569",
  "term_id": "GO:0000978",
  "gene": "UniProtKB:Q5MCW4",
  "gene_symbol": "ZNF569"
}